negative regulation of cardiac muscle adaptation [GO:0010616] (biological process) Definition: Any process that decreases the rate, extent or frequency of the process in which cardiac muscle adapts, with consequent modifications to structural and/or functional phenotypes, in response to a stimulus. Stimuli include contractile activity, loading conditions, substrate supply, and environmental factors. Sources: GOC:BHF, GOC:dph, GOC:tb Subtypes: negative regulation of cardiac muscle hypertrophy in response to stress [GO:1903243] Relationships: is a type of regulation of cardiac muscle adaptation [GO:0010612]; is a type of negative regulation of muscle adaptation [GO:0014745]; negatively regulates cardiac muscle adaptation [GO:0014887]